{
  "term_label": "Unknown molecular function",
  "gene_symbol": "MCC",
  "term_id": "UNKNOWN:0001",
  "gene_name": "Colorectal mutant cancer protein",
  "gene": "UniProtKB:P23508"
}